{
  "gene": "UniProtKB:P32418",
  "gene_name": "Sodium_calcium exchanger 1",
  "term_id": "GO:0006874",
  "gene_symbol": "SLC8A1",
  "term_label": "intracellular calcium ion homeostasis"
}